smooth muscle hyperplasia [GO:0014806] (biological process) Definition: A process, occurring in smooth muscle, in which there is an increase in cell number by cell division, often leading to an increase in the size of an organ. Relationships: is a type of smooth muscle adaptation [GO:0014805]; is a type of GO:0014900 Sources: GOC:mtg_muscle